{
  "term_label": "endoplasmic reticulum membrane",
  "gene_name": "Elongation of very long chain fatty acids protein 5",
  "gene_symbol": "ELOVL5",
  "term_id": "GO:0005789",
  "gene": "UniProtKB:Q9NYP7"
}